{
  "gene": "UniProtKB:Q9UBP9",
  "term_label": "Unknown cellular component",
  "term_id": "UNKNOWN:0003",
  "gene_name": "PTB domain-containing engulfment adapter protein 1",
  "gene_symbol": "GULP1"
}